{
  "term_label": "mitochondrion",
  "gene": "UniProtKB:Q16881",
  "term_id": "GO:0005739",
  "gene_symbol": "TXNRD1",
  "gene_name": "Thioredoxin reductase 1, cytoplasmic"
}